regulation of snRNA pseudouridine synthesis [GO:1905356] (biological process) Relationships: is a type of regulation of RNA metabolic process [GO:0051252]; regulates snRNA pseudouridine synthesis [GO:0031120] Subtypes: negative regulation of snRNA pseudouridine synthesis [GO:1905357], GO:1905358 Definition: Any process that modulates the frequency, rate or extent of snRNA pseudouridine synthesis. References: PMID:27268497 Sources: GOC:TermGenie, GO_REF:0000058